small-subunit processome assembly [GO:0034462] (biological process) Sources: GOC:mah Also known as: SSU processome assembly, small subunit processome assembly Relationships: is a type of protein-RNA complex assembly [GO:0022618]; BFO_0000050 cytosolic small ribosomal subunit assembly [GO:0180025] Definition: The aggregation, arrangement and bonding together of proteins and RNA molecules to form a small-subunit processome.